negative regulation of cellular response to oxidopamine [GO:1905847] (biological process) Definition: Any process that stops, prevents or reduces the frequency, rate or extent of cellular response to oxidopamine. Also known as: down regulation of cellular response to oxidopamine, down-regulation of cellular response to oxidopamine, downregulation of cellular response to oxidopamine, inhibition of cellular response to oxidopamine Relationships: is a type of negative regulation of cellular process [GO:0048523]; is a type of negative regulation of response to stimulus [GO:0048585]; is a type of regulation of cellular response to oxidopamine [GO:1905846]; negatively regulates cellular response to oxidopamine [GO:1905842] References: PMID:23721876 Sources: GOC:TermGenie, GO_REF:0000058